{
  "gene_name": "Cysteine protease ATG4A",
  "gene": "UniProtKB:Q8WYN0",
  "term_id": "GO:0000423",
  "term_label": "mitophagy",
  "gene_symbol": "ATG4A"
}